{
  "gene": "UniProtKB:O14974",
  "gene_name": "Protein phosphatase 1 regulatory subunit 12A",
  "gene_symbol": "PPP1R12A",
  "term_id": "GO:0030018",
  "term_label": "Z disc"
}